positive regulation of lysine biosynthetic process via alpha-aminoadipate and saccharopine [GO:2001196] (biological process) Definition: Any process that activates or increases the frequency, rate or extent of lysine biosynthetic process via alpha-aminoadipate and saccharopine. Relationships: is a type of positive regulation of small molecule metabolic process [GO:0062013]; is a type of positive regulation of amino acid biosynthetic process [GO:2000284]; is a type of regulation of lysine biosynthetic process via alpha-aminoadipate and saccharopine [GO:2001194]; positively regulates lysine biosynthetic process via alpha-aminoadipate and saccharopine [GO:0051975] Sources: GOC:obol Also known as: positive regulation of lysine biosynthesis via aminoadipic acid and saccharopine, positive regulation of lysine biosynthetic process via aminoadipic acid and saccharopine